{
  "gene_name": "Alpha_beta hydrolase domain-containing protein 17A",
  "gene": "UniProtKB:Q96GS6",
  "gene_symbol": "ABHD17A",
  "term_id": "GO:0099175",
  "term_label": "regulation of postsynapse organization"
}